{
  "gene": "UniProtKB:Q9Y2V0",
  "term_label": "nucleus",
  "term_id": "GO:0005634",
  "gene_symbol": "CDIN1",
  "gene_name": "CDAN1-interacting nuclease 1"
}